tRNA adenosine(64)-2'-O-ribosylphosphate transferase activity [GO:0043399] (molecular function) References: PMID:22030622, PMID:7954819 Sources: GOC:jl Relationships: is a type of pentosyltransferase activity [GO:0016763]; is a type of GO:0140101 Also known as: initiator tRNA phosphoribosyl-transferase activity, tRNA A64-2'-O-ribosylphosphate transferase activity Definition: Catalysis of the transfer of a phosphoribosyl group from 5'-phosphoribosyl-1'-pyrophosphate to position 64 of initiator tRNA.